{
  "gene": "UniProtKB:Q8NC69",
  "term_label": "cullin family protein binding",
  "gene_name": "BTB_POZ domain-containing protein KCTD6",
  "term_id": "GO:0097602",
  "gene_symbol": "KCTD6"
}